{
  "gene_name": "Exonuclease 1",
  "term_label": "DNA recombination",
  "term_id": "GO:0006310",
  "gene": "UniProtKB:Q9UQ84",
  "gene_symbol": "EXO1"
}